larval salivary gland morphogenesis [GO:0007436] (biological process) Relationships: is a type of GO:0007435; is a type of post-embryonic animal morphogenesis [GO:0009886]; is part of instar larval development [GO:0002168] Definition: The process, occurring in the larva, by which the anatomical structures of the salivary gland are generated and organized. Sources: GOC:jid